{
  "term_label": "Unknown molecular function",
  "term_id": "UNKNOWN:0001",
  "gene_name": "Heat shock protein beta-7",
  "gene": "UniProtKB:Q9UBY9",
  "gene_symbol": "HSPB7"
}